positive regulation of late stripe melanocyte differentiation [GO:0050950] (biological process) Definition: Any process that activates or increases the frequency, rate or extent of late stripe melanocyte differentiation. Sources: GOC:ai Also known as: positive regulation of late stripe melanophore differentiation, up regulation of late stripe melanocyte differentiation, up-regulation of late stripe melanocyte differentiation, upregulation of late stripe melanocyte differentiation, activation of late stripe melanocyte differentiation, stimulation of late stripe melanocyte differentiation Relationships: is a type of positive regulation of melanocyte differentiation [GO:0045636]; is a type of regulation of late stripe melanocyte differentiation [GO:0050940]; positively regulates late stripe melanocyte differentiation [GO:0050934]